{
  "term_id": "GO:0002062",
  "term_label": "chondrocyte differentiation",
  "gene_name": "Transcription factor SOX-9",
  "gene_symbol": "SOX9",
  "gene": "UniProtKB:P48436"
}